4-acetamidobutyrate deacetylase activity [GO:0047573] (molecular function) Also known as: 4-acetamidobutanoate amidohydrolase activity Sources: EC:3.5.1.63 Definition: Catalysis of the reaction: 4-acetamidobutanoate + H2O = acetate + 4-aminobutanoate. Relationships: is a type of hydrolase activity, acting on carbon-nitrogen (but not peptide) bonds, in linear amides [GO:0016811]; is a type of deacetylase activity [GO:0019213]